{
  "gene_name": "Olfactory receptor 1N1",
  "gene_symbol": "OR1N1",
  "term_label": "olfactory receptor activity",
  "term_id": "GO:0004984",
  "gene": "UniProtKB:Q8NGS0"
}